{
  "term_id": "UNKNOWN:0003",
  "term_label": "Unknown cellular component",
  "gene": "UniProtKB:Q96DE9",
  "gene_name": "Protein EOLA2",
  "gene_symbol": "EOLA2"
}